{
  "gene_symbol": "UGT1A4",
  "term_id": "GO:0004857",
  "term_label": "enzyme inhibitor activity",
  "gene": "UniProtKB:P22310",
  "gene_name": "UDP-glucuronosyltransferase 1A4"
}